{
  "gene": "UniProtKB:P45844",
  "gene_name": "ATP-binding cassette sub-family G member 1",
  "term_label": "cholesterol efflux",
  "term_id": "GO:0033344",
  "gene_symbol": "ABCG1"
}